{
  "term_id": "GO:0005615",
  "gene": "UniProtKB:P49863",
  "gene_symbol": "GZMK",
  "gene_name": "Granzyme K",
  "term_label": "extracellular space"
}